receptor-mediated endocytosis of virus by host cell [GO:0019065] (biological process) Definition: Any receptor-mediated endocytosis that is involved in the uptake of a virus into a host cell; successive instances of virus endocytosis result in the accumulation of virus particles within the cell. Subtypes: GO:0075512, caveolin-mediated endocytosis of virus by host cell [GO:0075513] Also known as: receptor mediated endocytosis by host of virus particle, receptor mediated endocytosis of virus by host, receptor mediated endocytosis of virus particle by host, receptor-mediated endocytosis of virus by host, viral receptor mediated endocytosis, virus receptor-mediated endocytosis by host, viral entry into host cell via receptor-mediated endocytosis Relationships: is a type of receptor-mediated endocytosis [GO:0006898]; is a type of endocytosis involved in viral entry into host cell [GO:0075509]; is part of symbiont entry into host cell [GO:0046718] Sources: GOC:bf, GOC:jl, ISBN:0781702534